galactose binding [GO:0005534] (molecular function) Relationships: is a type of GO:0048029 Sources: GOC:jl, ISBN:0198506732 Definition: Binding to aldohexose galactose (galacto-hexose), a common constituent of many oligo- and polysaccharides. Also known as: galactose binding lectin